{
  "gene": "UniProtKB:P49736",
  "gene_symbol": "MCM2",
  "term_id": "GO:0000727",
  "gene_name": "DNA replication licensing factor MCM2",
  "term_label": "double-strand break repair via break-induced replication"
}